{
  "gene_symbol": "GNL2",
  "term_label": "Unknown biological process",
  "gene_name": "Nucleolar GTP-binding protein 2",
  "gene": "UniProtKB:Q13823",
  "term_id": "UNKNOWN:0002"
}